{
  "gene_name": "Septin-4",
  "gene": "UniProtKB:O43236",
  "term_id": "GO:0061640",
  "term_label": "cytoskeleton-dependent cytokinesis",
  "gene_symbol": "SEPTIN4"
}